{
  "gene_name": "Mitochondrial calcium uniporter regulator 1",
  "gene": "UniProtKB:Q96AQ8",
  "term_label": "mitochondrial inner membrane",
  "term_id": "GO:0005743",
  "gene_symbol": "MCUR1"
}